{
  "gene": "UniProtKB:Q96RP9",
  "gene_symbol": "GFM1",
  "term_id": "GO:0003746",
  "term_label": "translation elongation factor activity",
  "gene_name": "Elongation factor G, mitochondrial"
}